sarcomerogenesis [GO:0048769] (biological process) Relationships: is a type of actomyosin structure organization [GO:0031032]; is part of myofibril assembly [GO:0030239] Also known as: myofibril production Definition: The process in which sarcomeres are added in series within a fiber. References: PMID:15947030 Sources: GOC:jid, GOC:lm